cellular response to Thyroid stimulating hormone [GO:1904401] (biological process) Definition: Any process that results in a change in state or activity of a cell (in terms of movement, secretion, enzyme production, gene expression, etc.) as a result of a Thyroid stimulating hormone stimulus. References: PMID:11238928 Sources: GOC:TermGenie, GO_REF:0000071 Relationships: is a type of response to Thyroid stimulating hormone [GO:1904400]; is a type of GO:1904588